response to radiation [GO:0009314] (biological process) Relationships: is a type of response to abiotic stimulus [GO:0009628] Sources: GOC:jl, Wikipedia:Electromagnetic_radiation Also known as: response to electromagnetic radiation stimulus, response to radiation stimulus Definition: Any process that results in a change in state or activity of a cell or an organism (in terms of movement, secretion, enzyme production, gene expression, etc.) as a result of an electromagnetic radiation stimulus. Electromagnetic radiation is a propagating wave in space with electric and magnetic components. These components oscillate at right angles to each other and to the direction of propagation. Note: Note that 'radiation' refers to electromagnetic radiation of any wavelength. Subtypes: GO:0009416, response to ionizing radiation [GO:0010212], cellular response to radiation [GO:0071478]